mitochondrial aspartyl-tRNA aminoacylation [GO:0070146] (BP) Definition: The process of coupling aspartate to aspartyl-tRNA in a mitochondrion, catalyzed by aspartyl-tRNA synthetase. In tRNA aminoacylation, the amino acid is first activated by linkage to AMP and then transferred to either the 2'- or the 3'-hydroxyl group of the 3'-adenosine residue of the tRNA. Relationships: is a type of aspartyl-tRNA aminoacylation [GO:0006422]; is_a tRNA aminoacylation for mitochondrial protein translation [GO:0070127] Sources: GOC:mah, GOC:mcc